{
  "gene_symbol": "ULK1",
  "gene_name": "Serine_threonine-protein kinase ULK1",
  "term_id": "GO:0000423",
  "term_label": "mitophagy",
  "gene": "UniProtKB:O75385"
}